{
  "term_label": "cytosol",
  "term_id": "GO:0005829",
  "gene_symbol": "GIGYF2",
  "gene_name": "GRB10-interacting GYF protein 2",
  "gene": "UniProtKB:Q6Y7W6"
}